indanol dehydrogenase activity [GO:0047718] (molecular function) Sources: EC:1.1.1.112, MetaCyc:INDANOL-DEHYDROGENASE-RXN Definition: Catalysis of the reaction: indan-1-ol + NAD(P)+ = indanone + NAD(P)H + H+. Relationships: is a type of oxidoreductase activity, acting on the CH-OH group of donors, NAD or NADP as acceptor [GO:0016616] Also known as: indan-1-ol:NAD(P)+ 1-oxidoreductase activity